{
  "term_id": "GO:0031145",
  "gene": "UniProtKB:Q86Y33",
  "gene_symbol": "CDC20B",
  "gene_name": "Cell division cycle protein 20 homolog B",
  "term_label": "anaphase-promoting complex-dependent catabolic process"
}